{
  "term_label": "cyclin-dependent protein kinase holoenzyme complex",
  "gene_name": "G2_mitotic-specific cyclin-B2",
  "gene_symbol": "CCNB2",
  "term_id": "GO:0000307",
  "gene": "UniProtKB:O95067"
}